{
  "gene_name": "Protein shisa-8",
  "gene_symbol": "SHISA8",
  "term_label": "postsynaptic membrane",
  "gene": "UniProtKB:B8ZZ34",
  "term_id": "GO:0045211"
}